beta-galactoside (CMP) alpha-2,3-sialyltransferase activity [GO:0003836] (molecular function) Definition: Catalysis of the reaction: CMP-N-acetylneuraminate + beta-D-galactosyl-(1->3)-N-acetyl-alpha-D-galactosaminyl-R = CMP + alpha-N-acetylneuraminyl-(2->3)-beta-D-galactosyl-(1->3)-N-acetyl-alpha-D-galactosaminyl-R. Sources: EC:2.4.3.4 Relationships: is a type of sialyltransferase activity [GO:0008373]